{
  "gene_symbol": "ERVH48-1",
  "term_label": "Unknown molecular function",
  "gene": "UniProtKB:M5A8F1",
  "gene_name": "Suppressyn",
  "term_id": "UNKNOWN:0001"
}